{
  "term_id": "UNKNOWN:0003",
  "term_label": "Unknown cellular component",
  "gene_symbol": "ANKAR",
  "gene": "UniProtKB:Q7Z5J8",
  "gene_name": "Ankyrin and armadillo repeat-containing protein"
}